regulation of protein localization to lysosome [GO:0150031] (biological process) Definition: Any process that modulates the frequency, rate or extent of protein localization to lysosome. Relationships: is a type of GO:0032880; RO_0002211 GO:0061462 References: PMID:24305806 Sources: GOC:aruk, GOC:bc Subtypes: positive regulation of protein localization to lysosome [GO:0150032], GO:0150033